histone H4K5 deacetylase activity, hydrolytic mechanism [GO:0180032] (molecular function) Also known as: histone H4K5 deacetylase activity References: PMID:37459529 Relationships: is a type of GO:0141051; is a type of histone deacetylase activity, hydrolytic mechanism [GO:0141221] Definition: Catalysis of the reaction: histone H4 N6-acetyl-L-lysine (position 5) + H2O = histone H4 L-lysine (position 5) + acetate. This reaction represents the removal of an acetyl group from lysine at position 5 of the histone H4 protein. Note: Note that the residue position corresponds to the canonical human H4 histone (UniProtKB:P02309); this residue is conserved across all eukaryotes. Note that the initiation methionine is cleaved, so the first residue is S1.